extrinsic component of periplasmic side of cell outer membrane [GO:0031245] (cellular component) Sources: GOC:dos, GOC:mah, GOC:mtg_sensu Relationships: is a type of GO:0031244; is part of periplasmic side of cell outer membrane [GO:0031241] Also known as: extrinsic to internal side of cell outer membrane, extrinsic to internal side of outer membrane, extrinsic to periplasmic side of cell outer membrane, extrinsic to internal leaflet of cell outer membrane Definition: The component of the cell outer membrane consisting of gene products and protein complexes that are loosely bound to periplasmic surface, but not integrated into the hydrophobic region.